{
  "gene": "UniProtKB:P50616",
  "gene_symbol": "TOB1",
  "term_id": "GO:0003714",
  "term_label": "transcription corepressor activity",
  "gene_name": "Protein Tob1"
}